carbon catabolite regulation of transcription from RNA polymerase II promoter [GO:0000429] (biological process) Relationships: is a type of GO:0006357; is a type of GO:0045990 Definition: A transcription regulation process in which the presence of one carbon source leads to the modulation of the frequency, rate, or extent of transcription, from an RNA polymerase II promoter, of specific genes involved in the metabolism of other carbon sources. Sources: GOC:krc, GOC:mah Also known as: regulation of transcription from RNA polymerase II promoter by carbon catabolites Subtypes: GO:0000430, GO:0000431, carbon catabolite activation of transcription from RNA polymerase II promoter [GO:0000436], GO:0000437, regulation of transcription from RNA polymerase II promoter by a nonfermentable carbon source [GO:0061413]